{
  "term_label": "G protein-coupled receptor signaling pathway",
  "term_id": "GO:0007186",
  "gene": "UniProtKB:Q6MZT1",
  "gene_name": "Regulator of G-protein signaling 7-binding protein",
  "gene_symbol": "RGS7BP"
}